{
  "gene_name": "T-box transcription factor T",
  "term_id": "GO:0001708",
  "gene_symbol": "TBXT",
  "term_label": "cell fate specification",
  "gene": "UniProtKB:O15178"
}